{
  "gene_symbol": "CPLX4",
  "gene": "UniProtKB:Q7Z7G2",
  "term_label": "SNARE complex",
  "term_id": "GO:0031201",
  "gene_name": "Complexin-4"
}